{
  "gene": "UniProtKB:P55160",
  "gene_symbol": "NCKAP1L",
  "term_label": "SCAR complex",
  "gene_name": "Nck-associated protein 1-like",
  "term_id": "GO:0031209"
}